{
  "term_label": "U2-type spliceosomal complex",
  "term_id": "GO:0005684",
  "gene": "UniProtKB:Q13435",
  "gene_name": "Splicing factor 3B subunit 2",
  "gene_symbol": "SF3B2"
}